regulation of methane biosynthetic process from dimethyl sulfide [GO:1900342] (biological process) Subtypes: negative regulation of methane biosynthetic process from dimethyl sulfide [GO:1900343], positive regulation of methane biosynthetic process from dimethyl sulfide [GO:1900344] Definition: Any process that modulates the frequency, rate or extent of methane biosynthetic process from dimethyl sulfide. Relationships: is a type of regulation of sulfur metabolic process [GO:0042762]; is_a regulation of cellular respiration [GO:0043457]; is a type of GO:1901577; regulates methane biosynthetic process from dimethyl sulfide [GO:2001131] Sources: GOC:TermGenie, GOC:mengo_curators